{
  "gene_symbol": "TOR1AIP1",
  "term_label": "nuclear membrane organization",
  "term_id": "GO:0071763",
  "gene": "UniProtKB:Q5JTV8",
  "gene_name": "Torsin-1A-interacting protein 1"
}